{
  "gene": "UniProtKB:P08218",
  "term_id": "GO:0005615",
  "term_label": "extracellular space",
  "gene_symbol": "CELA2B",
  "gene_name": "Chymotrypsin-like elastase family member 2B"
}